{
  "term_label": "synaptic transmission, glutamatergic",
  "gene_name": "Protein unc-13 homolog C",
  "term_id": "GO:0035249",
  "gene": "UniProtKB:Q8NB66",
  "gene_symbol": "UNC13C"
}